pseudopodium membrane [GO:0031260] (cellular component) Definition: The portion of the plasma membrane surrounding a pseudopodium. Sources: GOC:mah Relationships: is a type of cell projection membrane [GO:0031253]; is part of pseudopodium [GO:0031143]